{
  "gene": "UniProtKB:Q8IYW4",
  "gene_symbol": "ENTHD1",
  "term_label": "clathrin vesicle coat",
  "gene_name": "ENTH domain-containing protein 1",
  "term_id": "GO:0030125"
}